{
  "term_id": "UNKNOWN:0003",
  "gene": "UniProtKB:Q8N127",
  "gene_symbol": "OR5AS1",
  "gene_name": "Olfactory receptor 5AS1",
  "term_label": "Unknown cellular component"
}